{
  "term_label": "phagocytic vesicle",
  "gene": "UniProtKB:Q9BZG1",
  "gene_symbol": "RAB34",
  "term_id": "GO:0045335",
  "gene_name": "Ras-related protein Rab-34"
}